{
  "term_label": "Unknown biological process",
  "gene_name": "Retroelement silencing factor 1",
  "gene_symbol": "RESF1",
  "term_id": "UNKNOWN:0002",
  "gene": "UniProtKB:Q9HCM1"
}